interleukin-12 beta subunit binding [GO:0042163] (molecular function) Definition: Binding to the beta subunit of interleukin-12. Sources: GOC:mah Relationships: is a type of interleukin-12 binding [GO:0019972] Also known as: CLMFp40 binding, IL-12B binding, IL-12p40 binding, NKSFp40 binding